{
  "gene_name": "5-hydroxytryptamine receptor 2A",
  "term_label": "serotonin receptor signaling pathway",
  "term_id": "GO:0007210",
  "gene_symbol": "HTR2A",
  "gene": "UniProtKB:P28223"
}